aminoacyl-tRNA synthetase multienzyme complex [GO:0017101] (cellular component) Relationships: is a type of GO:0140535; is a type of catalytic complex [GO:1902494] References: PMID:16169847 Sources: GOC:jl Definition: A multienzyme complex found in all multicellular eukaryotes composed of eight proteins with aminoacyl-tRNA synthetase activities (abbreviated as: ArgRS, AspRS, GluProRS, GlnRS, IleRS, LeuRS, LysRS, MetRS where RS is the enzyme, preceded by the amino acid it uses as a substrate) as well as three non-synthetase proteins (p43, p38, and p18) with diverse functions. Several of these subunits are known dimers, so the total polypeptide count in the multisynthetase complex is at least fifteen. All of the enzymes in this assembly catalyze the same reaction, the covalent attachment of an amino acid to either the 2'- or 3'-hydroxyl of the 3'-terminal adenosine of tRNA, but using different substrates. Also known as: aminoacyl-tRNA synthetase complex, multisynthetase complex